ferulate catabolic process [GO:1901067] (biological process) Regulation: regulated by regulation of ferulate catabolic process [GO:1901466]; negatively regulated by negative regulation of ferulate catabolic process [GO:1901467]; positively regulated by positive regulation of ferulate catabolic process [GO:1901468] Sources: GOC:TermGenie, GOC:mengo_curators Relationships: is a type of phenol-containing compound catabolic process [GO:0019336]; is_a ferulate metabolic process [GO:0033494]; is a type of GO:0072329; is a type of olefinic compound catabolic process [GO:0120256]; is a type of ether catabolic process [GO:1901502] Definition: The chemical reactions and pathways resulting in the breakdown of ferulate. Also known as: ferulate breakdown, ferulate catabolism, ferulate degradation